{
  "gene": "UniProtKB:O60499",
  "gene_name": "Syntaxin-10",
  "term_id": "GO:0030672",
  "term_label": "synaptic vesicle membrane",
  "gene_symbol": "STX10"
}